neuron cellular homeostasis [GO:0070050] (biological process) Also known as: neuron maintenance Relationships: is a type of GO:0019725 Definition: The cellular homeostatic process that preserves a neuron in a stable, differentiated functional and structural state. Subtypes: synaptic vesicle lumen acidification [GO:0097401], GO:0099509 Sources: GOC:BHF, GOC:mah